{
  "gene": "UniProtKB:Q5VZ72",
  "gene_name": "Izumo sperm-egg fusion protein 3",
  "gene_symbol": "IZUMO3",
  "term_label": "Unknown biological process",
  "term_id": "UNKNOWN:0002"
}